{
  "term_id": "GO:0098609",
  "gene_name": "Roundabout homolog 2",
  "gene": "UniProtKB:Q9HCK4",
  "gene_symbol": "ROBO2",
  "term_label": "cell-cell adhesion"
}